pre-B cell differentiation [GO:0002329] (biological process) Relationships: is a type of immature B cell differentiation [GO:0002327] Also known as: pre-B lymphocyte differentiation, pre-B cell development Sources: GOC:jal, ISBN:0781735149 Note: Note that immunologists typically use the word 'development' to refer to cells of B or T cell lineages undergoing the process that GO describes as 'cell differentiation'. Definition: The process in which a precursor cell type acquires the specialized features of a pre-B cell. Pre-B cells follow the pro-B cell stage of immature B cell differentiation and undergo rearrangement of heavy chain V, D, and J gene segments.